{
  "gene": "UniProtKB:Q8NFR7",
  "term_label": "Unknown molecular function",
  "gene_name": "Coiled-coil domain-containing protein 148",
  "term_id": "UNKNOWN:0001",
  "gene_symbol": "CCDC148"
}